{
  "term_label": "cytosol",
  "gene_name": "Growth hormone receptor",
  "gene": "UniProtKB:P10912",
  "gene_symbol": "GHR",
  "term_id": "GO:0005829"
}